{
  "term_id": "UNKNOWN:0003",
  "term_label": "Unknown cellular component",
  "gene_symbol": "LINC03040",
  "gene": "UniProtKB:Q8N319",
  "gene_name": "Putative uncharacterized protein encoded by LINC03040"
}